ferredoxin-thioredoxin reductase activity [GO:0103012] (molecular function) Relationships: is a type of oxidoreductase activity, acting on a sulfur group of donors, iron-sulfur protein as acceptor [GO:0016673] References: PMID:14769790 Sources: GOC:pz, RHEA:42336 Also known as: ferredoxin:thioredoxin reductase activity Definition: Catalysis of the reaction: 2 H+ + 2 a reduced ferredoxin + an oxidized thioredoxin = 2 an oxidized ferredoxin + a reduced thioredoxin, involving a 4Fe-4S cluster and an adjacent active-site disulfide.